presynaptic cytosol [GO:0099523] (cellular component) Sources: GOC:dos Definition: The region of the cytosol consisting of all cytosol that is part of the presynapse. Relationships: is a type of GO:0099522; is part of presynapse [GO:0098793]